{
  "term_label": "Unknown biological process",
  "gene_symbol": "UNQ9165_PRO28630",
  "gene_name": "Putative uncharacterized protein UNQ9165_PRO28630",
  "term_id": "UNKNOWN:0002",
  "gene": "UniProtKB:Q6UXU0"
}